{
  "gene_symbol": "GSN",
  "gene": "UniProtKB:P06396",
  "term_id": "GO:0015629",
  "gene_name": "Gelsolin",
  "term_label": "actin cytoskeleton"
}